tricaffeoyl spermidine O-methyltransferase activity [GO:0102109] (molecular function) Relationships: is_a methyltransferase activity [GO:0008168] References: PMID:19077165 Sources: GOC:pz Definition: Catalysis of the reaction: tricaffeoyl spermidine + 3 S-adenosyl-L-methionine = 3 H+ + triferuloyl spermidine + 3 S-adenosyl-L-homocysteine.